{
  "gene": "UniProtKB:P32321",
  "term_label": "dUMP biosynthetic process",
  "term_id": "GO:0006226",
  "gene_name": "Deoxycytidylate deaminase",
  "gene_symbol": "DCTD"
}